{
  "gene": "UniProtKB:O75323",
  "term_label": "Unknown biological process",
  "gene_name": "Protein NipSnap homolog 2",
  "term_id": "UNKNOWN:0002",
  "gene_symbol": "NIPSNAP2"
}